{
  "gene_name": "Zinc transporter ZIP12",
  "gene": "UniProtKB:Q504Y0",
  "term_label": "plasma membrane",
  "term_id": "GO:0005886",
  "gene_symbol": "SLC39A12"
}